negative regulation of mRNA metabolic process [GO:1903312] (biological process) Also known as: down regulation of mRNA metabolic process, down regulation of mRNA metabolism, down-regulation of mRNA metabolic process, down-regulation of mRNA metabolism, downregulation of mRNA metabolic process, downregulation of mRNA metabolism, negative regulation of mRNA metabolism, inhibition of mRNA metabolic process, inhibition of mRNA metabolism Relationships: is a type of negative regulation of RNA metabolic process [GO:0051253]; is a type of regulation of mRNA metabolic process [GO:1903311]; negatively regulates GO:0016071 Subtypes: negative regulation of mRNA processing [GO:0050686], GO:0090367, negative regulation of mRNA catabolic process [GO:1902373] Sources: GOC:TermGenie, GOC:vw, GO_REF:0000058 Definition: Any process that stops, prevents or reduces the frequency, rate or extent of mRNA metabolic process.